{
  "term_id": "GO:0032591",
  "gene_symbol": "SHISA6",
  "gene": "UniProtKB:Q6ZSJ9",
  "term_label": "dendritic spine membrane",
  "gene_name": "Protein shisa-6"
}